{
  "term_id": "GO:0051020",
  "gene": "UniProtKB:Q5U651",
  "gene_name": "Ras-interacting protein 1",
  "gene_symbol": "RASIP1",
  "term_label": "GTPase binding"
}